histone H3K9me2/H3K9me3 demethylase activity [GO:0140684] (molecular function) Note: Comment: Note that the residue position corresponds to the canonical human H3 histone (UniProtKB:P84243); this residue is conserved across all eukaryotes. Residue 1 is the first residue following removal of the initiating Methionine (Met). Note that each histone is encoded by multiple genes, and sequences may vary across different genes within an organism. Relationships: is a type of 2-oxoglutarate-dependent dioxygenase activity [GO:0016706]; is a type of histone H3K9 demethylase activity [GO:0032454] Definition: Catalysis of the removal of a methyl group from a tri or a dimethyl-lysine residue at position 9 of the histone H3 protein. This is a dioxygenase reaction that is dependent on Fe(II) and 2-oxoglutarate. Also known as: histone H3K9me2 demethylase activity, histone H3-tri/dimethyl-lysine-9 demethylase activity, histone H3K9me3 demethylase activity References: PMID:20208542, PMID:20531378